{
  "gene_name": "[3-methyl-2-oxobutanoate dehydrogenase [lipoamide]] kinase, mitochondrial",
  "gene_symbol": "BCKDK",
  "term_label": "mitochondrion",
  "gene": "UniProtKB:O14874",
  "term_id": "GO:0005739"
}